{
  "term_id": "GO:0045211",
  "gene_name": "SH3 and multiple ankyrin repeat domains protein 3",
  "gene": "UniProtKB:Q9BYB0",
  "term_label": "postsynaptic membrane",
  "gene_symbol": "SHANK3"
}